manganese peroxidase activity [GO:0016689] (molecular function) Also known as: Mn(II):hydrogen-peroxide oxidoreductase activity, Mn-dependent (NADH-oxidizing) peroxidase activity, Mn-dependent peroxidase activity, peroxidase-M2 Sources: EC:1.11.1.13 Relationships: is a type of peroxidase activity [GO:0004601] Definition: Catalysis of the reaction: 2 Mn2+ + 2 H+ + hydrogen peroxide = 2 Mn3+ + 2 H2O.